alpha9-beta1 integrin-ADAM9 complex [GO:0071055] (cellular component) Also known as: ITGA9-ITGB1-ADAM9 complex References: PMID:11882657 Relationships: is a type of GO:0098797 Definition: A protein complex that consists of an alpha9-beta1 integrin complex bound to the transmembrane metallopeptidase ADAM9.